symbiont-mediated suppression of host dendritic cell mediated immune response [GO:0039673] (biological process) Sources: GOC:bf, GOC:jl, UniProtKB-KW:KW-1118 Relationships: is a type of symbiont-mediated perturbation of host innate immune response [GO:0052167] Also known as: modulation of host dendritic cell activity by virus, evasion by virus of host dendritic cell response, impairing dendritic cell function by virus, evasion by virus of host dendritic cell activity Definition: A process in which a symbiont inhibits or disrupts the dendritic cell mediated immune response of the host organism. The host is defined as the larger of the organisms involved in a symbiotic interaction.